{
  "term_label": "DNA-binding transcription factor activity",
  "term_id": "GO:0003700",
  "gene_symbol": "ZNF763",
  "gene": "UniProtKB:Q0D2J5",
  "gene_name": "Zinc finger protein 763"
}